type 2 melanin-concentrating hormone receptor binding [GO:0031778] (molecular function) Definition: Binding to a type 2 melanin-concentrating hormone receptor. Sources: GOC:mah, GOC:nln Also known as: type 2 melanin-concentrating hormone receptor ligand Relationships: is a type of GO:0031776